{
  "gene_name": "Urocortin",
  "term_id": "GO:2000252",
  "term_label": "negative regulation of feeding behavior",
  "gene": "UniProtKB:P55089",
  "gene_symbol": "UCN"
}